endonuclease complex [GO:1905348] (cellular component) Definition: A protein complex which is capable of endonuclease activity. Relationships: is a type of intracellular protein-containing complex [GO:0140535]; is a type of catalytic complex [GO:1902494] Note: An example of this is MUS81 in human (Q96NY9) in PMID:18413719 (inferred from direct assay). References: PMID:18413719 Sources: GOC:TermGenie, GOC:bhm, GO_REF:0000088 Subtypes: GO:1902555, endodeoxyribonuclease complex [GO:1905347]